{
  "gene_symbol": "ACSBG1",
  "gene": "UniProtKB:Q96GR2",
  "term_label": "long-chain fatty acid-CoA ligase activity",
  "gene_name": "Long-chain-fatty-acid--CoA ligase ACSBG1",
  "term_id": "GO:0004467"
}